{
  "gene_name": "DnaJ homolog subfamily C member 22",
  "gene": "UniProtKB:Q8N4W6",
  "term_label": "membrane",
  "gene_symbol": "DNAJC22",
  "term_id": "GO:0016020"
}